{
  "gene": "UniProtKB:O75150",
  "term_label": "nucleus",
  "gene_name": "E3 ubiquitin-protein ligase BRE1B",
  "term_id": "GO:0005634",
  "gene_symbol": "RNF40"
}